{
  "term_id": "UNKNOWN:0002",
  "gene_name": "Interleukin-17C",
  "term_label": "Unknown biological process",
  "gene": "UniProtKB:Q9P0M4",
  "gene_symbol": "IL17C"
}